{
  "gene_symbol": "ZNG1C",
  "gene_name": "Zinc-regulated GTPase metalloprotein activator 1C",
  "term_id": "GO:0005737",
  "term_label": "cytoplasm",
  "gene": "UniProtKB:Q5JTY5"
}